{
  "gene_name": "Staphylococcal nuclease domain-containing protein 1",
  "term_id": "GO:0006402",
  "gene_symbol": "SND1",
  "term_label": "mRNA catabolic process",
  "gene": "UniProtKB:Q7KZF4"
}